{
  "term_id": "GO:0000209",
  "gene_symbol": "STUB1",
  "term_label": "protein polyubiquitination",
  "gene_name": "E3 ubiquitin-protein ligase CHIP",
  "gene": "UniProtKB:Q9UNE7"
}